{
  "term_label": "ATPase-coupled intramembrane lipid transporter activity",
  "gene": "UniProtKB:O60312",
  "gene_name": "Phospholipid-transporting ATPase VA",
  "term_id": "GO:0140326",
  "gene_symbol": "ATP10A"
}